sarcosine oxidase activity [GO:0008115] (molecular function) Definition: Catalysis of the reaction: H2O + O2 + sarcosine = formaldehyde + glycine + H2O2. Also known as: sarcosine:oxygen oxidoreductase (demethylating) Relationships: is a type of GO:0016647 Sources: EC:1.5.3.1, RHEA:13313